{
  "term_label": "G protein-coupled receptor signaling pathway",
  "gene_name": "G-protein coupled receptor 55",
  "gene": "UniProtKB:Q9Y2T6",
  "gene_symbol": "GPR55",
  "term_id": "GO:0007186"
}